{
  "gene_symbol": "PMAIP1",
  "term_label": "mitochondrion",
  "gene": "UniProtKB:Q13794",
  "gene_name": "Phorbol-12-myristate-13-acetate-induced protein 1",
  "term_id": "GO:0005739"
}